{
  "gene_symbol": "UPF3B",
  "term_id": "GO:0045727",
  "gene": "UniProtKB:Q9BZI7",
  "term_label": "positive regulation of translation",
  "gene_name": "Regulator of nonsense transcripts 3B"
}